UDP-N-acetyl-D-glucosamine:N-acetylmuramoyl-L-alanyl-D-glutamyl-meso-2,6-diaminopimelyl-D-alanyl-D-alanine-diphosphoundecaprenol 4-beta-N-acetylglucosaminlytransferase activity [GO:0051991] (molecular function) Relationships: is a type of acetylglucosaminyltransferase activity [GO:0008375] Definition: Catalysis of the reaction: di-trans-octa-cis-undecaprenyl diphospho-N-acetyl-alpha-D-muramoyl-L-alanyl-D-glutamyl-meso-2,6-diaminopimeloyl-D-alanyl-D-alanine + UDP-N-acetyl-alpha-D-glucosamine = di-trans-octa-cis-undecaprenyl diphospho-[N-acetyl-alpha-D-glucosaminyl-(1->4)]-N-acetyl-alpha-D-muramoyl-L-alanyl-D-glutamyl-meso-2,6-diaminopimeloyl-D-alanyl-D-alanine + H+ + UDP. Sources: RHEA:31227